{
  "term_label": "Unknown cellular component",
  "gene_name": "Putative uncharacterized protein LINC02875",
  "term_id": "UNKNOWN:0003",
  "gene": "UniProtKB:Q86X59",
  "gene_symbol": "LINC02875"
}